succinate-CoA ligase complex (ADP-forming) [GO:0009361] (cellular component) Relationships: is a type of succinate-CoA ligase complex [GO:0042709] References: PMID:9874242 Sources: GOC:jl Also known as: succinyl-CoA synthetase, ADP-forming Definition: A heterodimeric enzyme complex, composed of an alpha and beta chain, most usually found in (but not limited to) bacteria. Functions in the TCA cycle, hydrolyzing succinyl-CoA into succinate and CoA, thereby forming ATP.